{
  "gene_name": "Nuclear factor of activated T-cells 5",
  "gene_symbol": "NFAT5",
  "gene": "UniProtKB:O94916",
  "term_id": "GO:0045944",
  "term_label": "positive regulation of transcription by RNA polymerase II"
}